{
  "gene_symbol": "LYZL2",
  "term_id": "GO:0003796",
  "gene": "UniProtKB:Q7Z4W2",
  "gene_name": "Lysozyme-like protein 2",
  "term_label": "lysozyme activity"
}